{
  "gene": "UniProtKB:P62304",
  "gene_name": "Small nuclear ribonucleoprotein E",
  "term_id": "UNKNOWN:0001",
  "gene_symbol": "SNRPE",
  "term_label": "Unknown molecular function"
}